{
  "gene_name": "Integrin alpha-7",
  "gene_symbol": "ITGA7",
  "term_id": "GO:0038023",
  "term_label": "signaling receptor activity",
  "gene": "UniProtKB:Q13683"
}